reflex [GO:0060004] (BP) Definition: An automatic response to a stimulus beginning with a nerve impulse from a receptor and ending with the action of an effector such as a gland or a muscle. Signaling never reaches a level of consciousness. Relationships: is a type of response to external stimulus [GO:0009605] Subtypes: proboscis extension reflex [GO:0007637], musculoskeletal movement, spinal reflex action [GO:0050883], vestibular reflex [GO:0060005], righting reflex [GO:0060013], eye blink reflex [GO:0060082], GO:0060156, pilomotor reflex [GO:0097195], sneeze reflex [GO:0160023] Sources: GOC:dph, ISBN:0877797099